{
  "gene_name": "HLA class II histocompatibility antigen, DM beta chain",
  "term_label": "late endosome membrane",
  "term_id": "GO:0031902",
  "gene_symbol": "HLA-DMB",
  "gene": "UniProtKB:P28068"
}